trehalose transmembrane transporter activity [GO:0015574] (molecular function) Subtypes: protein-N(PI)-phosphohistidine-trehalose phosphotransferase system transporter activity [GO:0022879], trehalose:proton symporter activity [GO:0044693] Definition: Enables the transfer of trehalose from one side of a membrane to the other. Trehalose is the disaccharide alpha-D-glucopyranosyl-alpha-D-glucopyranoside that acts of a reserve carbohydrate in certain fungi, algae and lichens. Sources: GOC:mtg_transport, ISBN:0198506732, ISBN:0815340729 Relationships: is a type of GO:0015154; is part of trehalose transport [GO:0015771] Also known as: trehalose permease activity